symbiont-mediated suppression of host toll-like receptor signaling pathway [GO:0039722] (biological process) Definition: A process in which a symbiont interferes with, inhibits or disrupts a toll-like receptor signaling pathway in the host organism. The host is defined as the larger of the organisms involved in a symbiotic interaction. Relationships: is a type of symbiont-mediated suppression of host signal transduction pathway [GO:0052029] Also known as: inhibition of host TLR pathway by virus, suppression by virus of host TLR signaling pathway, suppression by virus of host toll-like receptor signaling pathway References: PMID:15944308, PMID:17299722, PMID:18327267